{
  "gene_symbol": "TMEM44",
  "term_id": "GO:0015174",
  "gene_name": "Transmembrane protein 44",
  "term_label": "basic amino acid transmembrane transporter activity",
  "gene": "UniProtKB:Q2T9K0"
}